{
  "gene_symbol": "KIR2DS4",
  "term_label": "immune response-inhibiting cell surface receptor signaling pathway",
  "gene_name": "Killer cell immunoglobulin-like receptor 2DS4",
  "gene": "UniProtKB:P43632",
  "term_id": "GO:0002767"
}